{
  "gene": "UniProtKB:O75791",
  "gene_symbol": "GRAP2",
  "term_label": "signal transduction",
  "gene_name": "GRB2-related adapter protein 2",
  "term_id": "GO:0007165"
}